granaticin biosynthetic process [GO:1901109] (biological process) Also known as: granaticin anabolism, granaticin biosynthesis, granaticin formation, granaticin synthesis Relationships: is a type of polyketide biosynthetic process [GO:0030639]; is a type of ketone biosynthetic process [GO:0042181] Sources: GOC:TermGenie, GOC:yaf, UniPathway:UPA00175 Definition: The chemical reactions and pathways resulting in the formation of granaticin.